{
  "gene_name": "Metallothionein-1M",
  "term_label": "cellular response to copper ion",
  "gene_symbol": "MT1M",
  "gene": "UniProtKB:Q8N339",
  "term_id": "GO:0071280"
}